{
  "gene": "UniProtKB:Q8IZR5",
  "gene_name": "CKLF-like MARVEL transmembrane domain-containing protein 4",
  "term_label": "Unknown molecular function",
  "term_id": "UNKNOWN:0001",
  "gene_symbol": "CMTM4"
}